{
  "gene_symbol": "ZNFX1",
  "gene_name": "NFX1-type zinc finger-containing protein 1",
  "term_id": "GO:0031048",
  "term_label": "regulatory ncRNA-mediated heterochromatin formation",
  "gene": "UniProtKB:Q9P2E3"
}